{
  "term_id": "UNKNOWN:0002",
  "gene": "UniProtKB:Q6ZQQ2",
  "term_label": "Unknown biological process",
  "gene_name": "Spermatogenesis-associated protein 31D1",
  "gene_symbol": "SPATA31D1"
}